N-acetylgalactosamine transport [GO:0015763] (biological process) Sources: GOC:ai Relationships: is a type of carbohydrate derivative transport [GO:1901264] Definition: The directed movement of N-acetylgalactosamine into, out of or within a cell, or between cells, by means of some agent such as a transporter or pore. N-acetylgalactosamine, 2-acetamido-2-deoxygalactopyranose, is the n-acetyl derivative of galactosamine.